{
  "gene": "UniProtKB:O00141",
  "term_id": "GO:0035556",
  "gene_symbol": "SGK1",
  "term_label": "intracellular signal transduction",
  "gene_name": "Serine_threonine-protein kinase Sgk1"
}